{
  "gene_symbol": "SRC",
  "term_id": "GO:2001237",
  "gene": "UniProtKB:P12931",
  "term_label": "negative regulation of extrinsic apoptotic signaling pathway",
  "gene_name": "Proto-oncogene tyrosine-protein kinase Src"
}